{
  "gene_symbol": "PERCC1",
  "gene": "UniProtKB:A0A1W2PR82",
  "term_label": "Unknown molecular function",
  "gene_name": "Protein PERCC1",
  "term_id": "UNKNOWN:0001"
}